{
  "term_id": "GO:0002720",
  "gene_symbol": "CLEC7A",
  "gene_name": "C-type lectin domain family 7 member A",
  "term_label": "positive regulation of cytokine production involved in immune response",
  "gene": "UniProtKB:Q9BXN2"
}